{
  "gene_symbol": "CHRNA1",
  "term_label": "synaptic transmission, cholinergic",
  "term_id": "GO:0007271",
  "gene": "UniProtKB:P02708",
  "gene_name": "Acetylcholine receptor subunit alpha"
}